{
  "term_label": "nerve growth factor receptor binding",
  "gene_symbol": "NGF",
  "gene": "UniProtKB:P01138",
  "term_id": "GO:0005163",
  "gene_name": "Beta-nerve growth factor"
}